radial glial cell fate commitment in forebrain [GO:0022023] (BP) Relationships: is a type of glial cell fate commitment [GO:0021781]; is a type of commitment of multipotent stem cells to neuronal lineage in forebrain [GO:0021898]; is part of forebrain radial glial cell differentiation [GO:0021861] Definition: The process in which the developmental fate of a cell becomes restricted such that it will develop into a radial glial cell in the forebrain. Sources: GOC:cls, GOC:dgh, GOC:dph, GOC:jid, GO_REF:0000021